glucosamine catabolic process [GO:0006043] (biological process) Sources: GOC:jl, ISBN:0198506732 Definition: The chemical reactions and pathways resulting in the breakdown of glucosamine (2-amino-2-deoxyglucopyranose), an aminodeoxysugar that occurs in combined form in chitin. Relationships: is_a glucosamine metabolic process [GO:0006041]; is a type of glucosamine-containing compound catabolic process [GO:1901072] Also known as: chitosamine catabolic process, chitosamine catabolism, glucosamine breakdown, glucosamine catabolism, glucosamine degradation